{
  "gene": "UniProtKB:P20700",
  "term_id": "GO:0005652",
  "term_label": "nuclear lamina",
  "gene_name": "Lamin-B1",
  "gene_symbol": "LMNB1"
}